exopeptidase activity [GO:0008238] (molecular function) Relationships: is a type of peptidase activity [GO:0008233] Also known as: exoprotease activity Sources: https://www.ebi.ac.uk/merops/about/glossary.shtml#EXOPEPTIDASE Subtypes: aminopeptidase activity [GO:0004177], carboxypeptidase activity [GO:0004180], metalloexopeptidase activity [GO:0008235], dipeptidyl-peptidase activity [GO:0008239], peptidyl-dipeptidase activity [GO:0008241], dipeptidase activity [GO:0016805], tripeptidase activity [GO:0034701], GO:0070004, serine-type exopeptidase activity [GO:0070008], eoxin E4 synthase activity [GO:0097263] Definition: Catalysis of the hydrolysis of a peptide bond not more than three residues from the N- or C-terminus of a polypeptide chain, in a reaction that requires a free N-terminal amino group, C-terminal carboxyl group or both.